UDP-D-galactose metabolic process [GO:0052573] (biological process) Relationships: is a type of GO:0009225 Subtypes: UDP-galactose biosynthetic process [GO:0052574] Also known as: UDP-D-galactopyranose metabolic process, UDP-D-galactopyranose metabolism, UDP-D-galactose metabolism, UDP-galactose metabolic process, UDP-galactose metabolism, uridine diphosphate galactose metabolic process, uridine diphosphate galactose metabolism Sources: GOC:ai Definition: The chemical reactions and pathways involving UDP-D-galactose, a substance composed of D-galactose in glycosidic linkage with guanosine diphosphate.